opioid growth factor receptor activity [GO:0140625] (molecular function) Definition: Combining with the opioid growth factor (OGF, met-enkephalin) and transmitting the signal across the nuclear membrane. Met-enkephalin is an endogenous opioid peptide that binds to opioid and opioid growth factor receptors, regulating tissue growth in a variety of cellular processes. References: PMID:11890982 Also known as: methionine enkephalin receptor activity, met-enkephalin receptor activity, metenkefalin receptor activity Relationships: is_a peptide receptor activity [GO:0001653]